pole plasm mitochondrial rRNA localization [GO:0019095] (biological process) Subtypes: pole plasm mitochondrial lrRNA localization [GO:0019096], pole plasm mitochondrial srRNA localization [GO:0019097] Definition: Any process in which mitochondrial ribosomal RNA is transported to, or maintained in, the oocyte pole plasm. An example of this is found in Drosophila melanogaster. Sources: ISBN:0879694238 Relationships: is a type of pole plasm RNA localization [GO:0007316]; is a type of mitochondrial RNA localization [GO:0019093] Also known as: establishment and maintenance of mitochondrial rRNA localization in pole plasm, oocyte pole plasm mitochondrial rRNA localization, pole plasm mitochondrial rRNA localisation